{
  "gene": "UniProtKB:Q6MZM0",
  "gene_name": "Ferroxidase HEPHL1",
  "gene_symbol": "HEPHL1",
  "term_label": "plasma membrane",
  "term_id": "GO:0005886"
}